{
  "gene": "UniProtKB:O00743",
  "gene_symbol": "PPP6C",
  "term_label": "G1/S transition of mitotic cell cycle",
  "term_id": "GO:0000082",
  "gene_name": "Serine_threonine-protein phosphatase 6 catalytic subunit"
}